{
  "term_id": "GO:0009897",
  "term_label": "external side of plasma membrane",
  "gene_name": "Butyrophilin-like protein 8",
  "gene": "UniProtKB:Q6UX41",
  "gene_symbol": "BTNL8"
}